{
  "term_id": "GO:0043518",
  "term_label": "negative regulation of DNA damage response, signal transduction by p53 class mediator",
  "gene_name": "HLA class II histocompatibility antigen gamma chain",
  "gene_symbol": "CD74",
  "gene": "UniProtKB:P04233"
}